cellular response to dexamethasone stimulus [GO:0071549] (biological process) Sources: GOC:mah, GOC:yaf Relationships: is a type of cellular response to glucocorticoid stimulus [GO:0071385]; is a type of GO:0071548; is_a cellular response to ketone [GO:1901655] Definition: Any process that results in a change in state or activity of a cell (in terms of movement, secretion, enzyme production, gene expression, etc.) as a result of a dexamethasone stimulus.